{
  "gene_symbol": "GLYAT",
  "term_label": "glycine N-acyltransferase activity",
  "gene_name": "Glycine N-acyltransferase",
  "term_id": "GO:0047961",
  "gene": "UniProtKB:Q6IB77"
}